type-II dockerin domain binding [GO:1990309] (molecular function) Definition: Binding to a type-II dockerin domain of a protein. Type-II dockerin domain is the binding partner of type-II cohesin domain. References: PMID:23195689, PMID:24080387 Sources: GOC:mengo_curators Relationships: is a type of GO:0019904